{
  "gene_symbol": "LINC02902",
  "term_id": "UNKNOWN:0001",
  "gene": "UniProtKB:Q6ZTY9",
  "gene_name": "Putative uncharacterized protein LINC02902",
  "term_label": "Unknown molecular function"
}